{
  "gene": "UniProtKB:Q562F6",
  "gene_symbol": "SGO2",
  "term_label": "kinetochore",
  "gene_name": "Shugoshin 2",
  "term_id": "GO:0000776"
}